{
  "term_label": "transmembrane transporter binding",
  "gene_name": "Sodium channel subunit beta-4",
  "term_id": "GO:0044325",
  "gene_symbol": "SCN4B",
  "gene": "UniProtKB:Q8IWT1"
}